{
  "term_label": "Unknown biological process",
  "gene_symbol": "ITLN2",
  "gene_name": "Intelectin-2",
  "gene": "UniProtKB:Q8WWU7",
  "term_id": "UNKNOWN:0002"
}